{
  "gene": "UniProtKB:P35916",
  "gene_name": "Vascular endothelial growth factor receptor 3",
  "gene_symbol": "FLT4",
  "term_label": "positive regulation of MAPK cascade",
  "term_id": "GO:0043410"
}